positive regulation of interleukin-2-mediated signaling pathway [GO:1902207] (biological process) Definition: Any process that activates or increases the frequency, rate or extent of interleukin-2-mediated signaling pathway. References: PMID:11909529 Sources: GOC:TermGenie Also known as: positive regulation of IL-2-mediated signaling pathway, positive regulation of interleukin-2-mediated signalling pathway, up regulation of IL-2-mediated signaling pathway, up regulation of interleukin-2-mediated signaling pathway, up regulation of interleukin-2-mediated signalling pathway, up-regulation of IL-2-mediated signaling pathway, up-regulation of interleukin-2-mediated signaling pathway, up-regulation of interleukin-2-mediated signalling pathway, upregulation of IL-2-mediated signaling pathway, upregulation of interleukin-2-mediated signaling pathway, upregulation of interleukin-2-mediated signalling pathway, activation of IL-2-mediated signaling pathway, activation of interleukin-2-mediated signaling pathway, activation of interleukin-2-mediated signalling pathway Relationships: is a type of positive regulation of cytokine-mediated signaling pathway [GO:0001961]; is a type of regulation of interleukin-2-mediated signaling pathway [GO:1902205]; positively regulates interleukin-2-mediated signaling pathway [GO:0038110]